{
  "term_label": "microtubule severing",
  "gene_name": "Katanin p60 ATPase-containing subunit A-like 2",
  "gene_symbol": "KATNAL2",
  "gene": "UniProtKB:Q8IYT4",
  "term_id": "GO:0051013"
}